{
  "term_label": "DNA-binding transcription factor activity, RNA polymerase II-specific",
  "term_id": "GO:0000981",
  "gene_symbol": "EN2",
  "gene": "UniProtKB:P19622",
  "gene_name": "Homeobox protein engrailed-2"
}